testicular fusome organization [GO:0030724] (biological process) Definition: A process that is carried out at the cellular level which results in the assembly, arrangement of constituent parts, or disassembly of the fusome of testicular cells, an organelle derived from the spectrosome. Relationships: is a type of GO:0045478; is part of spermatogenesis [GO:0007283] Sources: GOC:dph, GOC:jl, GOC:mah, ISBN:0879694238 Also known as: testicular fusome organisation, testicular fusome organization and biogenesis